{
  "term_id": "GO:0061630",
  "term_label": "ubiquitin protein ligase activity",
  "gene_symbol": "TRIM11",
  "gene_name": "E3 ubiquitin-protein ligase TRIM11",
  "gene": "UniProtKB:Q96F44"
}